{
  "term_id": "GO:0000978",
  "term_label": "RNA polymerase II cis-regulatory region sequence-specific DNA binding",
  "gene_name": "snRNA-activating protein complex subunit 4",
  "gene_symbol": "SNAPC4",
  "gene": "UniProtKB:Q5SXM2"
}